tetrapeptide transmembrane transporter activity [GO:1901584] (molecular function) Relationships: is a type of GO:0035673; BFO_0000050 GO:1901583 Definition: Enables the transfer of tetrapeptide from one side of a membrane to the other. Sources: GOC:TermGenie